{
  "gene": "UniProtKB:Q8N119",
  "term_label": "metalloendopeptidase activity",
  "gene_name": "Matrix metalloproteinase-21",
  "term_id": "GO:0004222",
  "gene_symbol": "MMP21"
}